{
  "gene": "UniProtKB:P55345",
  "gene_name": "Protein arginine N-methyltransferase 2",
  "term_label": "histone methyltransferase activity",
  "gene_symbol": "PRMT2",
  "term_id": "GO:0042054"
}